positive regulation of eosinophil migration [GO:2000418] (biological process) Relationships: is a type of positive regulation of leukocyte migration [GO:0002687]; is a type of regulation of eosinophil migration [GO:2000416]; positively regulates GO:0072677 Subtypes: positive regulation of eosinophil extravasation [GO:2000421], GO:2000424 Definition: Any process that activates or increases the frequency, rate or extent of eosinophil migration. Sources: GOC:mah